regulation of motor neuron migration [GO:1905483] (biological process) Definition: Any process that modulates the frequency, rate or extent of motor neuron migration. References: PMID:16516839 Sources: GOC:TermGenie, GO_REF:0000058 Relationships: is a type of regulation of neuron migration [GO:2001222]; regulates motor neuron migration [GO:0097475] Subtypes: regulation of lateral motor column neuron migration [GO:1902076], negative regulation of motor neuron migration [GO:1905484], positive regulation of motor neuron migration [GO:1905485]